{
  "term_label": "negative regulation of DNA-templated transcription",
  "gene_symbol": "SFMBT2",
  "term_id": "GO:0045892",
  "gene_name": "Scm-like with four MBT domains protein 2",
  "gene": "UniProtKB:Q5VUG0"
}